{
  "gene_symbol": "SMPD2",
  "term_id": "GO:0071944",
  "gene": "UniProtKB:O60906",
  "gene_name": "Sphingomyelin phosphodiesterase 2",
  "term_label": "cell periphery"
}